{
  "gene_name": "Neuroglobin",
  "term_label": "oxygen binding",
  "gene": "UniProtKB:Q9NPG2",
  "term_id": "GO:0019825",
  "gene_symbol": "NGB"
}